negative regulation of oligodendrocyte progenitor proliferation [GO:0070446] (biological process) Definition: Any process that stops or decreases the rate or extent of oligodendrocyte progenitor proliferation. Sources: GOC:mah, GOC:sl Relationships: is a type of negative regulation of gliogenesis [GO:0014014]; is a type of regulation of oligodendrocyte progenitor proliferation [GO:0070445]; is a type of GO:2000178; negatively regulates oligodendrocyte progenitor proliferation [GO:0070444] Also known as: negative regulation of oligodendrocyte precursor proliferation